regulation of hair follicle placode formation [GO:0061168] (biological process) Sources: GOC:dph Definition: Any process that modulates the rate, frequency, or extent of hair follicle placode formation, the developmental process in which a hair placode forms. An hair follicle placode is a thickening of the ectoderm that will give rise to the hair follicle bud. Subtypes: positive regulation of hair placode formation [GO:0061169], negative regulation of hair follicle placode formation [GO:0061170] Relationships: is a type of regulation of anatomical structure morphogenesis [GO:0022603]; regulates GO:0060789